{
  "gene_name": "Taste receptor type 2 member 50",
  "gene": "UniProtKB:P59544",
  "term_label": "membrane",
  "term_id": "GO:0016020",
  "gene_symbol": "TAS2R50"
}